{
  "term_id": "GO:0014069",
  "gene": "UniProtKB:Q9UPX8",
  "gene_name": "SH3 and multiple ankyrin repeat domains protein 2",
  "gene_symbol": "SHANK2",
  "term_label": "postsynaptic density"
}